specification of floral organ number [GO:0048833] (biological process) Subtypes: GO:0048834 Definition: Any process that modulates the number of floral organs formed in a floral whorl. Sources: GOC:tb Relationships: is a type of developmental process involved in reproduction [GO:0003006]; is a type of specification of plant organ number [GO:0048832]; is part of flower development [GO:0009908]